lead ion transmembrane transporter activity [GO:0015094] (MF) Sources: GOC:ai Also known as: zinc, cadmium, cobalt, nickel, lead-efflux ATPase activity Relationships: is a type of metal ion transmembrane transporter activity [GO:0046873]; is part of lead ion transport [GO:0015692] Definition: Enables the transfer of lead (Pb) ions from one side of a membrane to the other.